{
  "gene_name": "M-phase inducer phosphatase 2",
  "term_label": "protein tyrosine phosphatase activity",
  "gene": "UniProtKB:P30305",
  "term_id": "GO:0004725",
  "gene_symbol": "CDC25B"
}